{
  "term_label": "very long-chain fatty acid catabolic process",
  "gene": "UniProtKB:P33897",
  "gene_name": "ATP-binding cassette sub-family D member 1",
  "gene_symbol": "ABCD1",
  "term_id": "GO:0042760"
}